homogentisate prenyltransferase activity [GO:0010354] (molecular function) Definition: Catalysis of the transfer of a prenyl group from one compound (donor) to homogentisic acid. Subtypes: homogentisate phytyltransferase activity [GO:0010176], homogentisate farnesyltransferase activity [GO:0010355], homogentisate geranylgeranyltransferase activity [GO:0010356], GO:0010357 Relationships: is a type of prenyltransferase activity [GO:0004659] References: PMID:16989822